{
  "gene": "UniProtKB:P10073",
  "term_id": "UNKNOWN:0003",
  "gene_symbol": "ZSCAN22",
  "term_label": "Unknown cellular component",
  "gene_name": "Zinc finger and SCAN domain-containing protein 22"
}